{
  "gene_name": "SERTA domain-containing protein 4",
  "gene_symbol": "SERTAD4",
  "gene": "UniProtKB:Q9NUC0",
  "term_label": "Unknown cellular component",
  "term_id": "UNKNOWN:0003"
}